biotin carboxylase activity [GO:0004075] (molecular function) Sources: EC:6.3.4.14 Relationships: is_a ligase activity, forming carbon-nitrogen bonds [GO:0016879] Also known as: biotin carboxylase (component of acetyl CoA carboxylase) activity, biotin-carboxyl-carrier-protein:carbon-dioxide ligase (ADP-forming) activity Definition: Catalysis of the reaction: ATP + biotin-carboxyl-carrier protein + CO2 = ADP + phosphate + carboxybiotin-carboxyl-carrier protein.